regulation of inner ear receptor cell differentiation [GO:2000980] (biological process) Subtypes: regulation of inner ear auditory receptor cell differentiation [GO:0045607], negative regulation of inner ear receptor cell differentiation [GO:2000981], GO:2000982 Sources: GOC:obol Relationships: is a type of regulation of mechanoreceptor differentiation [GO:0045631]; regulates inner ear receptor cell differentiation [GO:0060113] Also known as: regulation of inner ear hair cell differentiation Definition: Any process that modulates the frequency, rate or extent of inner ear receptor cell differentiation.